telomeric D-loop binding [GO:0061821] (molecular function) Definition: Binding to a telomeric D-loop. A telomeric D-loop is a three-stranded DNA displacement loop that forms at the site where the telomeric 3' single-stranded DNA overhang (formed of the repeat sequence TTAGGG in mammals) is tucked back inside the double-stranded component of telomeric DNA molecule, thus forming a t-loop or telomeric-loop and protecting the chromosome terminus. Relationships: is a type of D-loop DNA binding [GO:0062037] References: PMID:19734539 Sources: GOC:BHF, GOC:BHF_telomere, GOC:nc Also known as: telomeric Displacement-loop binding